alpha-1,3-mannosylglycoprotein 2-beta-N-acetylglucosaminyltransferase activity [GO:0003827] (molecular function) Definition: Catalysis of the reaction: 3-(alpha-D-mannosyl)-beta-D-mannosyl-R + UDP-N-acetyl-alpha-D-glucosamine = 3-(2-[N-acetyl-beta-D-glucosaminyl]-alpha-D-mannosyl)-beta-D-mannosyl-R + H+ + UDP. Sources: EC:2.4.1.101, RHEA:11456 Also known as: alpha-1,3-mannosylglycoprotein beta-1,2-N-acetylglucosaminyltransferase activity, GNTI activity, GnTI, N-acetylglucosaminyltransferase I activity, N-glycosyl-oligosaccharide-glycoprotein N-acetylglucosaminyltransferase I activity, UDP-N-acetyl-D-glucosamine:3-(alpha-D-mannosyl)-beta-D-mannosyl-glycoprotein 2-beta-N-acetyl-D-glucosaminyltransferase activity, UDP-N-acetylglucosaminyl:alpha-1,3-D-mannoside-beta-1,2-N-acetylglucosaminyltransferase I activity, UDP-N-acetylglucosaminyl:alpha-3-D-mannoside beta-1,2-N-acetylglucosaminyltransferase I activity, alpha-1,3-mannosyl-glycoprotein 2-beta-N-acetylglucosaminyltransferase activity, alpha-1,3-mannosyl-glycoprotein beta-1,2-N-acetylglucosaminyltransferase activity, uridine diphosphoacetylglucosamine-alpha-1,3-mannosylglycoprotein beta-1,2-N-acetylglucosaminyltransferase activity Relationships: is a type of acetylglucosaminyltransferase activity [GO:0008375]; is a type of catalytic activity, acting on a glycoprotein [GO:0140103]